{
  "gene_symbol": "PDE2A",
  "term_label": "negative regulation of cAMP/PKA signal transduction",
  "gene_name": "cGMP-dependent 3',5'-cyclic phosphodiesterase",
  "gene": "UniProtKB:O00408",
  "term_id": "GO:0141162"
}